{
  "term_id": "GO:0031751",
  "term_label": "D4 dopamine receptor binding",
  "gene_symbol": "CLIC6",
  "gene_name": "Chloride intracellular channel protein 6",
  "gene": "UniProtKB:Q96NY7"
}